{
  "gene_symbol": "GKN1",
  "term_label": "regulation of cell population proliferation",
  "gene_name": "Gastrokine-1",
  "term_id": "GO:0042127",
  "gene": "UniProtKB:Q9NS71"
}